{
  "term_id": "GO:0004984",
  "gene_name": "Olfactory receptor 2Y1",
  "gene": "UniProtKB:Q8NGV0",
  "gene_symbol": "OR2Y1",
  "term_label": "olfactory receptor activity"
}